{
  "gene_symbol": "ZNF273",
  "gene_name": "Zinc finger protein 273",
  "term_label": "regulation of DNA-templated transcription",
  "term_id": "GO:0006355",
  "gene": "UniProtKB:Q14593"
}